podocyte apoptotic process [GO:1903210] (biological process) Definition: Any apoptotic process in a glomerular visceral epithelial cell. References: PMID:23515840 Sources: GOC:TermGenie, GO_REF:0000085 Also known as: glomerular podocyte apoptotic process, glomerular visceral epithelial cell apoptotic process, glomerular podocyte apoptosis, glomerular visceral epithelial cell apoptosis, podocyte apoptosis Relationships: is a type of epithelial cell apoptotic process [GO:1904019] Regulation: regulated by regulation of podocyte apoptotic process [GO:1904633]; negatively regulated by negative regulation of podocyte apoptotic process [GO:1904634]; positively regulated by positive regulation of podocyte apoptotic process [GO:1904635]